{
  "gene": "UniProtKB:Q8TEZ7",
  "term_id": "GO:0003707",
  "term_label": "nuclear steroid receptor activity",
  "gene_name": "Membrane progestin receptor beta",
  "gene_symbol": "PAQR8"
}